fusion of virus membrane with host endosome membrane [GO:0039654] (biological process) Also known as: fusion of virus membrane with host endosomal membrane, viral entry into host cell via caveolae-mediated endocytosis followed by membrane fusion with the endosome membrane, viral entry into host cell via caveolin-mediated endocytosis followed by membrane fusion with the endosome membrane, viral entry into host cell via clathrin-mediated endocytosis followed by membrane fusion with the endosome membrane, viral penetration via endocytosis followed by caveolae-mediated membrane fusion with the endosome membrane, viral penetration via endocytosis followed by clathrin-mediated membrane fusion with the endosome membrane, viral entry into host cell via endocytosis followed by membrane fusion with host endosome, viral entry into host cell via endocytosis followed by membrane fusion with the endosome membrane Definition: Fusion of a virus membrane with a host endosome membrane. Occurs after internalization of the virus through the endosomal pathway, and results in release of the virus contents into the cell. Relationships: is a type of GO:0039663 Subtypes: fusion of virus membrane with host macropinosome membrane [GO:0075503] Sources: GOC:bf, UniProtKB-KW:KW-1170, VZ:992